positive regulation of proteasomal ubiquitin-dependent protein catabolic process [GO:0032436] (biological process) Relationships: is a type of regulation of proteasomal ubiquitin-dependent protein catabolic process [GO:0032434]; is a type of positive regulation of proteasomal protein catabolic process [GO:1901800]; is a type of positive regulation of ubiquitin-dependent protein catabolic process [GO:2000060]; positively regulates proteasome-mediated ubiquitin-dependent protein catabolic process [GO:0043161] Subtypes: positive regulation of SCF-dependent proteasomal ubiquitin-dependent catabolic process [GO:0062027], positive regulation of anaphase-promoting complex-dependent catabolic process [GO:1905786] Definition: Any process that activates or increases the frequency, rate or extent of the breakdown of a protein or peptide by hydrolysis of its peptide bonds, initiated by the covalent attachment of ubiquitin, and mediated by the proteasome. Sources: GOC:mah Also known as: up regulation of proteasomal ubiquitin-dependent protein catabolic process, up-regulation of proteasomal ubiquitin-dependent protein catabolic process, upregulation of proteasomal ubiquitin-dependent protein catabolic process, activation of proteasomal ubiquitin-dependent protein catabolic process, stimulation of proteasomal ubiquitin-dependent protein catabolic process